{
  "gene_name": "Transmembrane protein 82",
  "gene": "UniProtKB:A0PJX8",
  "term_label": "Unknown cellular component",
  "term_id": "UNKNOWN:0003",
  "gene_symbol": "TMEM82"
}